{
  "term_id": "GO:0035735",
  "gene": "UniProtKB:A0AVF1",
  "gene_name": "Intraflagellar transport protein 56",
  "term_label": "intraciliary transport involved in cilium assembly",
  "gene_symbol": "IFT56"
}